peptidyl-L-beta-methylthioaspartic acid biosynthetic process from peptidyl-aspartic acid [GO:0018339] (biological process) Relationships: is a type of GO:0018197; is a type of GO:0018198 Sources: RESID:AA0232 Also known as: peptidyl-L-beta-methylthioaspartic acid anabolism from peptidyl-aspartic acid, peptidyl-L-beta-methylthioaspartic acid formation from peptidyl-aspartic acid, peptidyl-L-beta-methylthioaspartic acid synthesis from peptidyl-aspartic acid, peptidyl-aspartic acid methylthiolation Definition: The modification of peptidyl-aspartic acid to form peptidyl-L-beta-methylthioaspartic acid, typical of bacterial ribosomal protein S12.